{
  "term_label": "Unknown cellular component",
  "term_id": "UNKNOWN:0003",
  "gene": "UniProtKB:P42768",
  "gene_symbol": "WAS",
  "gene_name": "Actin nucleation-promoting factor WAS"
}